{
  "gene_name": "cAMP-dependent protein kinase catalytic subunit gamma",
  "term_label": "protein kinase A regulatory subunit binding",
  "gene_symbol": "PRKACG",
  "gene": "UniProtKB:P22612",
  "term_id": "GO:0034237"
}